{
  "term_id": "GO:0000423",
  "gene": "UniProtKB:Q9C0C7",
  "gene_name": "Activating molecule in BECN1-regulated autophagy protein 1",
  "term_label": "mitophagy",
  "gene_symbol": "AMBRA1"
}